{
  "term_id": "GO:0003823",
  "gene_name": "Immunoglobulin heavy variable 3-66",
  "term_label": "antigen binding",
  "gene": "UniProtKB:A0A0C4DH42",
  "gene_symbol": "IGHV3-66"
}